gamma-aminobutyric acid secretion [GO:0014051] (biological process) Also known as: GABA secretion Definition: The regulated release of gamma-aminobutyric acid by a cell or a tissue. The gamma-aminobutyric acid is the principal inhibitory neurotransmitter in the brain but is also found in several extraneural tissues. Regulation: regulated by GO:0014052; negatively regulated by negative regulation of gamma-aminobutyric acid secretion [GO:0014053]; positively regulated by GO:0014054 Relationships: is a type of gamma-aminobutyric acid transport [GO:0015812]; is a type of acid secretion [GO:0046717] Subtypes: gamma-aminobutyric acid secretion, neurotransmission [GO:0061534] Sources: GOC:ef